{
  "gene_name": "Mitogen-activated protein kinase kinase kinase 7",
  "gene_symbol": "MAP3K7",
  "term_label": "Unknown cellular component",
  "gene": "UniProtKB:O43318",
  "term_id": "UNKNOWN:0003"
}